{
  "gene_symbol": "UBL4B",
  "gene": "UniProtKB:Q8N7F7",
  "term_label": "Unknown biological process",
  "term_id": "UNKNOWN:0002",
  "gene_name": "Ubiquitin-like protein 4B"
}